{
  "term_id": "GO:0007186",
  "gene": "UniProtKB:Q8NGG2",
  "term_label": "G protein-coupled receptor signaling pathway",
  "gene_symbol": "OR5T2",
  "gene_name": "Olfactory receptor 5T2"
}